Golgi vesicle docking [GO:0048211] (biological process) Definition: The initial attachment of a Golgi transport vesicle membrane to a target membrane, mediated by proteins protruding from the membrane of the Golgi vesicle and the target membrane. References: PMID:10219233 Sources: GOC:jid, ISBN:0716731363 Relationships: is a type of vesicle docking [GO:0048278]; is part of Golgi vesicle transport [GO:0048193] Also known as: Golgi vesicle docking with target membrane, Golgi vesicle to membrane docking, Golgi-derived vesicle docking, dictyosome vesicle docking to target membrane